{
  "gene_symbol": "RTN3",
  "gene_name": "Reticulon-3",
  "gene": "UniProtKB:O95197",
  "term_label": "endoplasmic reticulum tubular network formation",
  "term_id": "GO:0071787"
}